{
  "term_label": "regulation of cell shape",
  "term_id": "GO:0008360",
  "gene_name": "Radixin",
  "gene_symbol": "RDX",
  "gene": "UniProtKB:P35241"
}